3-hydroxyanthranilate 4-C-methyltransferase activity [GO:0030767] (molecular function) Relationships: is a type of S-adenosylmethionine-dependent methyltransferase activity [GO:0008757] Also known as: 3-hydroxyanthranilate 4-methyltransferase activity, S-adenosyl-L-methionine:3-hydroxyanthranilate 4-C-methyltransferase activity Definition: Catalysis of the reaction: 3-hydroxyanthranilate + S-adenosyl-L-methionine = 3-hydroxy-4-methylanthranilate + S-adenosyl-L-homocysteine + H+. Sources: EC:2.1.1.97, RHEA:17833